{
  "gene_symbol": "SHANK2",
  "gene_name": "SH3 and multiple ankyrin repeat domains protein 2",
  "gene": "UniProtKB:Q9UPX8",
  "term_label": "associative learning",
  "term_id": "GO:0008306"
}